{
  "gene_name": "Krueppel-like factor 17",
  "term_label": "regulation of transcription by RNA polymerase II",
  "gene": "UniProtKB:Q5JT82",
  "gene_symbol": "KLF17",
  "term_id": "GO:0006357"
}